{
  "term_label": "protein ubiquitination",
  "gene_name": "E3 ubiquitin-protein ligase MIB2",
  "gene": "UniProtKB:Q96AX9",
  "term_id": "GO:0016567",
  "gene_symbol": "MIB2"
}